negative regulation of double-strand break repair via nonhomologous end joining [GO:2001033] (biological process) Relationships: is a type of GO:2000780; is a type of regulation of double-strand break repair via nonhomologous end joining [GO:2001032]; negatively regulates double-strand break repair via nonhomologous end joining [GO:0006303] Definition: Any process that stops, prevents or reduces the frequency, rate or extent of double-strand break repair via nonhomologous end joining. Also known as: negative regulation of NHEJ Sources: GOC:obol